{
  "gene_symbol": "NXF2B",
  "term_id": "GO:0003723",
  "term_label": "RNA binding",
  "gene": "UniProtKB:Q9GZY0",
  "gene_name": "Nuclear RNA export factor 2"
}